high molecular weight kininogen receptor binding [GO:0030987] (MF) Definition: Binding to a high molecular weight kininogen receptor. Relationships: is a type of GO:0005102 Sources: GOC:mah